{
  "gene": "UniProtKB:Q9BYR9",
  "gene_symbol": "KRTAP2-4",
  "gene_name": "Keratin-associated protein 2-4",
  "term_label": "Unknown molecular function",
  "term_id": "UNKNOWN:0001"
}